{
  "gene_symbol": "PHC3",
  "term_id": "GO:0003682",
  "term_label": "chromatin binding",
  "gene": "UniProtKB:Q8NDX5",
  "gene_name": "Polyhomeotic-like protein 3"
}